{
  "term_id": "UNKNOWN:0003",
  "gene_symbol": "MEI1",
  "term_label": "Unknown cellular component",
  "gene": "UniProtKB:Q5TIA1",
  "gene_name": "Meiosis inhibitor protein 1"
}